phosphoarginine catabolic process [GO:0046313] (biological process) Sources: GOC:ai Relationships: is a type of phosphagen catabolic process [GO:0042397]; is a type of L-amino acid catabolic process [GO:0170035]; is a type of non-proteinogenic amino acid catabolic process [GO:0170044] Definition: The chemical reactions and pathways resulting in the breakdown of phosphoarginine, a phosphorylated derivative of the amino acid arginine. Also known as: phosphoarginine breakdown, phosphoarginine catabolism, phosphoarginine degradation